MH2 domain binding [GO:0035500] (molecular function) Definition: Binding to a MH2 (MAD homology 2) protein domain. The MH2 domain is found at the carboxy-terminus of MAD related proteins such as Smads. The MH2 domain mediates interaction with a wide variety of proteins and provides specificity and selectivity to Smad function and also is critical for mediating interactions in Smad oligomers. Sources: GOC:curators Also known as: MAD homology 2 domain binding Relationships: is a type of protein domain specific binding [GO:0019904]